{
  "term_label": "microtubule nucleation",
  "gene_symbol": "TUBGCP2",
  "term_id": "GO:0007020",
  "gene_name": "Gamma-tubulin complex component 2",
  "gene": "UniProtKB:Q9BSJ2"
}